{
  "gene_symbol": "PIWIL4",
  "gene_name": "Piwi-like protein 4",
  "term_label": "piRNA processing",
  "term_id": "GO:0034587",
  "gene": "UniProtKB:Q7Z3Z4"
}